{
  "term_id": "UNKNOWN:0001",
  "gene_name": "Protein YIPF6",
  "gene": "UniProtKB:Q96EC8",
  "gene_symbol": "YIPF6",
  "term_label": "Unknown molecular function"
}